{
  "gene_symbol": "TTF1",
  "gene": "UniProtKB:Q15361",
  "gene_name": "Transcription termination factor 1",
  "term_id": "GO:0006363",
  "term_label": "termination of RNA polymerase I transcription"
}